{
  "term_label": "protein serine/threonine kinase activity",
  "term_id": "GO:0004674",
  "gene_symbol": "CDKL1",
  "gene": "UniProtKB:Q00532",
  "gene_name": "Cyclin-dependent kinase-like 1"
}